{
  "gene": "UniProtKB:Q5VXM1",
  "gene_name": "CUB domain-containing protein 2",
  "gene_symbol": "CDCP2",
  "term_id": "UNKNOWN:0002",
  "term_label": "Unknown biological process"
}